mitochondrial electron transport, cytochrome c to oxygen [GO:0006123] (biological process) Sources: ISBN:0716731363 Definition: The transfer of electrons from cytochrome c to oxygen that occurs during oxidative phosphorylation, mediated by the multisubunit enzyme known as complex IV. Relationships: is a type of aerobic electron transport chain [GO:0019646]; is part of mitochondrial ATP synthesis coupled electron transport [GO:0042775] Also known as: complex IV (reduction of O2)